{
  "gene": "UniProtKB:Q8N3I7",
  "term_id": "GO:0036064",
  "gene_name": "Bardet-Biedl syndrome 5 protein",
  "term_label": "ciliary basal body",
  "gene_symbol": "BBS5"
}